chromosomal 5-methylcytosine DNA demethylation, direct 5-methylcytosine excision pathway [GO:0141169] (biological process) Relationships: is a type of chromosomal 5-methylcytosine DNA demethylation pathway [GO:0141166] Also known as: epigenetic 5-methylcytosine DNA demethylation, direct 5-methylcytosine excision pathway Regulation: positively regulated by positive regulation of 5-methylcytosine DNA demethylation, direct 5-methylcytosine excision pathway [GO:0141170] Definition: An epigenetic cytosine DNA demethylation pathway that involves a DNA glycosylase that directly excises 5-methylcytosine (5-meC) to initiate its replacement with unmethylated cytosine through base excision repair. This pathway is known to occur in plants. In addition to CG sites, plants also methylate cytosines within CHH and CNG sequences. References: PMID:21862972, PMID:31546611, PMID:36478523 Note: Note that this term describes one of the biochemical pathways of chromosomal cytosine demethylation but is agnostic to the effect on gene expression. If the data supports it, consider co-annotating to 'positive regulation of gene expression, epigenetic ; GO:0044029' or a child.